endocardial cushion cell development [GO:0061444] (biological process) Relationships: is a type of cardiac cell development [GO:0055006]; is part of endocardial cushion cell differentiation [GO:0061443] Sources: GOC:BHF, GOC:dph Definition: The process whose specific outcome is the progression of an endocardial cushion cell over time, from its formation to the mature state.